follicular fluid formation in ovarian follicle antrum involved in fused antrum stage [GO:0003003] (biological process) Definition: The ovulation cycle process in which one central cavity separating the oocyte/cumulus complex from mural granulosa and theca cells is formed as part of the fused antrum stage of oogenesis. Sources: GOC:dph, GOC:isa_complete Also known as: follicular fluid formation in ovarian follicle antrum during fused antrum stage Relationships: is a type of follicular fluid formation in ovarian follicle antrum [GO:0001548]; is part of fused antrum stage [GO:0048165]